{
  "gene": "UniProtKB:O60259",
  "gene_name": "Kallikrein-8",
  "gene_symbol": "KLK8",
  "term_label": "extracellular space",
  "term_id": "GO:0005615"
}